{
  "gene_name": "Ectonucleoside triphosphate diphosphohydrolase 4",
  "term_id": "GO:0005794",
  "gene_symbol": "ENTPD4",
  "term_label": "Golgi apparatus",
  "gene": "UniProtKB:Q9Y227"
}